{
  "term_label": "DNA-binding transcription factor activity, RNA polymerase II-specific",
  "term_id": "GO:0000981",
  "gene": "UniProtKB:Q6PG37",
  "gene_name": "Zinc finger protein 790",
  "gene_symbol": "ZNF790"
}